{
  "gene_name": "Extracellular calcium-sensing receptor",
  "term_label": "intracellular calcium ion homeostasis",
  "gene": "UniProtKB:P41180",
  "term_id": "GO:0006874",
  "gene_symbol": "CASR"
}